{
  "gene_symbol": "ACE",
  "term_id": "GO:0002003",
  "gene": "UniProtKB:P12821",
  "term_label": "angiotensin maturation",
  "gene_name": "Angiotensin-converting enzyme"
}